{
  "gene_symbol": "RPS6KA6",
  "term_id": "GO:0030330",
  "gene": "UniProtKB:Q9UK32",
  "term_label": "DNA damage response, signal transduction by p53 class mediator",
  "gene_name": "Ribosomal protein S6 kinase alpha-6"
}